macrophage activation [GO:0042116] (biological process) Definition: A change in morphology and behavior of a macrophage resulting from exposure to a cytokine, chemokine, cellular ligand, or soluble factor. References: PMID:14506301 Sources: GOC:mgi_curators, ISBN:0781735149 Also known as: macrophage polarization Relationships: is_a myeloid leukocyte activation [GO:0002274] Subtypes: microglial cell activation [GO:0001774], macrophage activation involved in immune response [GO:0002281] Regulation: regulated by regulation of macrophage activation [GO:0043030]; negatively regulated by GO:0043031; positively regulated by positive regulation of macrophage activation [GO:0043032]